{
  "gene": "UniProtKB:Q8IZA3",
  "gene_name": "Histone H1.8",
  "term_label": "chromosome condensation",
  "gene_symbol": "H1-8",
  "term_id": "GO:0030261"
}